{
  "term_id": "UNKNOWN:0003",
  "gene": "UniProtKB:A0A494C1I1",
  "gene_symbol": "LOC728392",
  "gene_name": "Uncharacterized protein",
  "term_label": "Unknown cellular component"
}